sensory perception of taste [GO:0050909] (biological process) Subtypes: sensory perception of bitter taste [GO:0050913], sensory perception of salty taste [GO:0050914], GO:0050915, sensory perception of sweet taste [GO:0050916], sensory perception of umami taste [GO:0050917] Also known as: gustation, sense of taste, taste, taste perception Relationships: is a type of GO:0007606 Sources: GOC:ai Definition: The series of events required for an organism to receive a gustatory stimulus, convert it to a molecular signal, and recognize and characterize the signal. Gustation involves the direct detection of chemical composition, usually through contact with chemoreceptor cells. This is a neurological process.